inner plaque of mitotic spindle pole body [GO:0061497] (cellular component) Definition: One of three laminate structures that form the mitotic spindle pole body; the inner plaque is in the nucleus. Sources: GOC:dph, GOC:vw Relationships: is_a inner plaque of spindle pole body [GO:0005822]; is part of mitotic spindle pole body [GO:0044732]